{
  "gene": "UniProtKB:A4UGR9",
  "gene_name": "Xin actin-binding repeat-containing protein 2",
  "term_id": "GO:0005925",
  "gene_symbol": "XIRP2",
  "term_label": "focal adhesion"
}